{
  "gene_name": "Small integral membrane protein 10",
  "term_id": "UNKNOWN:0003",
  "term_label": "Unknown cellular component",
  "gene": "UniProtKB:Q96HG1",
  "gene_symbol": "SMIM10"
}